histone pre-mRNA stem-loop binding [GO:0071207] (molecular function) Relationships: is_a pre-mRNA binding [GO:0036002] Definition: Binding to a conserved stem-loop structure found in histone pre-mRNAs. References: PMID:19470752